slow muscle cell migration [GO:1904969] (biological process) Also known as: slow-twitch muscle cell migration Relationships: is a type of myotube cell migration [GO:0110122] Definition: The orderly movement of a slow muscle cell from one site to another. Note: The directional migration of a slow muscle cell from one site to another within the embryo. References: PMID:14667409, PMID:15572133, PMID:25534553 Sources: GOC:TermGenie, GOC:ymb, GO_REF:0000091